protein phosphate-linked glycosylation [GO:0042076] (biological process) Relationships: is a type of glycoprotein biosynthetic process [GO:0009101] References: PMID:7499424 Definition: The glycosylation of peptidyl-amino acids through a phosphoester bond forming, for example, GlcNAc-alpha-1-P-Ser residues. Also known as: phosphoglycosylation, protein amino acid phosphate-linked glycosylation